{
  "gene": "UniProtKB:Q96MT8",
  "term_id": "GO:0007099",
  "gene_symbol": "CEP63",
  "term_label": "centriole replication",
  "gene_name": "Centrosomal protein of 63 kDa"
}